{
  "term_label": "plasma membrane",
  "gene": "UniProtKB:A0A1B0GTQ4",
  "term_id": "GO:0005886",
  "gene_name": "Protein myomixer",
  "gene_symbol": "MYMX"
}